{
  "term_label": "Unknown molecular function",
  "gene_symbol": "PRIM2",
  "term_id": "UNKNOWN:0001",
  "gene": "UniProtKB:P49643",
  "gene_name": "DNA primase large subunit"
}